{
  "gene_name": "Testis-expressed protein 30",
  "gene": "UniProtKB:Q5JUR7",
  "gene_symbol": "TEX30",
  "term_id": "UNKNOWN:0002",
  "term_label": "Unknown biological process"
}